{
  "term_id": "UNKNOWN:0002",
  "gene_name": "Putative uncharacterized protein FLJ45355",
  "gene": "UniProtKB:Q6ZSN1",
  "gene_symbol": "Q6ZSN1",
  "term_label": "Unknown biological process"
}